{
  "gene_name": "Fatty acid-binding protein, adipocyte",
  "gene_symbol": "FABP4",
  "gene": "UniProtKB:P15090",
  "term_label": "fatty acid binding",
  "term_id": "GO:0005504"
}